{
  "gene": "UniProtKB:F8VTS6",
  "gene_name": "Ret finger protein-like 4A-like protein 1",
  "term_label": "regulation of gene expression",
  "term_id": "GO:0010468",
  "gene_symbol": "RFPL4AL1"
}